RNAi-mediated antiviral immunity against DNA virus [GO:0051215] (biological process) Also known as: DNA VIGS, DNA virus induced gene silencing, DNA virus-induced PTGS, DNA virus-induced gene silencing References: PMID:15165191, PMID:17693253, PMID:23151511 Relationships: is a type of GO:0009616 Definition: An RNAi-mediated post-transcriptional gene silencing pathway induced by DNA viruses leading to a sequence-specific degradation of target mRNAs or inhibition of translation. In plants, DCL3 is the primary Dicer to detect DNA viruses.